alkanesulfonate biosynthetic process [GO:0046305] (biological process) Subtypes: GO:0042412 Definition: The chemical reactions and pathways resulting in the formation of alkanesulfonates, the anion of alkanesulfonic acids, sulfonic acid derivatives containing an aliphatic hydrocarbon group. Also known as: alkanesulfonate anabolism, alkanesulfonate biosynthesis, alkanesulfonate formation, alkanesulfonate synthesis, alkanesulphonate biosynthesis, alkanesulphonate biosynthetic process Relationships: is a type of GO:0016053; is_a GO:0019694; is a type of sulfur compound biosynthetic process [GO:0044272] Sources: GOC:ai